{
  "term_id": "GO:0051087",
  "term_label": "protein-folding chaperone binding",
  "gene_name": "Prostaglandin E synthase 3",
  "gene": "UniProtKB:Q15185",
  "gene_symbol": "PTGES3"
}